{
  "gene_symbol": "BCL2",
  "term_id": "GO:0001836",
  "term_label": "release of cytochrome c from mitochondria",
  "gene": "UniProtKB:P10415",
  "gene_name": "Apoptosis regulator Bcl-2"
}